ferrichrome biosynthetic process [GO:0031169] (biological process) Sources: GOC:mah, ISBN:0198506732 Relationships: is a type of hydroxymate-containing siderophore biosynthetic process [GO:0019539]; is a type of amide biosynthetic process [GO:0043604] Subtypes: ferricrocin biosynthetic process [GO:0031171] Also known as: ferrichrome anabolism, ferrichrome biosynthesis, ferrichrome formation, ferrichrome synthesis, ferrichrome biosynthetic process, peptide formation, ferrichrome biosynthetic process, peptide modification Regulation: regulated by regulation of ferrichrome biosynthetic process [GO:1905568]; RO_0002212 by negative regulation of ferrichrome biosynthetic process [GO:1905569]; positively regulated by positive regulation of ferrichrome biosynthetic process [GO:1905570] Definition: The chemical reactions and pathways resulting in the formation of a ferrichrome. Ferrichromes are any of a group of growth-promoting Fe(III) chelates formed by various genera of microfungi. They are homodetic cyclic hexapeptides made up of a tripeptide of glycine (or other small neutral amino acids) and a tripeptide of an N'acyl-N4-hydroxy-L-ornithine.